{
  "term_label": "cytoplasm",
  "gene_name": "5-formyltetrahydrofolate cyclo-ligase",
  "gene": "UniProtKB:P49914",
  "gene_symbol": "MTHFS",
  "term_id": "GO:0005737"
}